{
  "term_id": "UNKNOWN:0003",
  "gene": "UniProtKB:Q96M53",
  "gene_symbol": "TBATA",
  "term_label": "Unknown cellular component",
  "gene_name": "Protein TBATA"
}